relaxation of skeletal muscle [GO:0090076] (biological process) Sources: GOC:BHF, GOC:rl Relationships: is a type of relaxation of muscle [GO:0090075] Definition: A process in which the extent of skeletal muscle tissue contraction is reduced. Muscle relaxation involves the removal of calcium from the cytoplasm to the sarcoplasmic reticulum lumen through the action of Ca2+ ATPases.